ribulokinase activity [GO:0008741] (molecular function) Sources: EC:2.7.1.16 Relationships: is a type of phosphotransferase activity, alcohol group as acceptor [GO:0016773]; is a type of carbohydrate kinase activity [GO:0019200] Definition: Catalysis of the reaction: ATP + L(or D)-ribulose = ADP + L(or D)-ribulose 5-phosphate. Also known as: L-ribulokinase activity, ATP:L(or D)-ribulose 5-phosphotransferase activity, ribulokinase (phosphorylating)